outer medullary collecting duct development [GO:0072060] (biological process) Definition: The process whose specific outcome is the progression of the outer medullary collecting duct over time, from its formation to the mature structure. The outer medullary collecting duct is the portion of the collecting duct that lies in the renal outer medulla. Sources: GOC:mtg_kidney_jan10 Relationships: is a type of collecting duct development [GO:0072044]